regulation of natural killer cell chemotaxis [GO:2000501] (biological process) Sources: GOC:BHF Definition: Any process that modulates the frequency, rate or extent of natural killer cell chemotaxis. Relationships: is a type of regulation of lymphocyte chemotaxis [GO:1901623]; regulates natural killer cell chemotaxis [GO:0035747] Subtypes: negative regulation of natural killer cell chemotaxis [GO:2000502], positive regulation of natural killer cell chemotaxis [GO:2000503]